{
  "gene_name": "Paraneoplastic antigen-like protein 6A",
  "term_id": "UNKNOWN:0003",
  "gene_symbol": "PNMA6A",
  "gene": "UniProtKB:P0CW24",
  "term_label": "Unknown cellular component"
}